{
  "gene_symbol": "RNF148",
  "gene": "UniProtKB:Q8N7C7",
  "term_id": "GO:0006511",
  "gene_name": "RING finger protein 148",
  "term_label": "ubiquitin-dependent protein catabolic process"
}